{
  "gene_name": "Bridge-like lipid transfer protein family member 3A",
  "gene": "UniProtKB:Q6BDS2",
  "gene_symbol": "BLTP3A",
  "term_id": "UNKNOWN:0002",
  "term_label": "Unknown biological process"
}